{
  "term_id": "GO:0005634",
  "gene_symbol": "APOBEC3D",
  "term_label": "nucleus",
  "gene_name": "DNA dC-dU-editing enzyme APOBEC-3D",
  "gene": "UniProtKB:Q96AK3"
}